neuron projection development [GO:0031175] (biological process) Definition: The process whose specific outcome is the progression of a neuron projection over time, from its formation to the mature structure. A neuron projection is any process extending from a neural cell, such as axons or dendrites (collectively called neurites). Also known as: neurite biosynthesis, neurite development, neurite formation, neurite growth, neurite outgrowth Sources: GOC:mah Regulation: regulated by regulation of neuron projection development [GO:0010975]; positively regulated by GO:0010976; negatively regulated by negative regulation of neuron projection development [GO:0010977] Relationships: is a type of plasma membrane bounded cell projection organization [GO:0120036]; is part of GO:0048666 Subtypes: retrograde extension [GO:0003389], dendrite development [GO:0016358], neuron projection regeneration [GO:0031102], inner ear receptor cell stereocilium organization [GO:0060122], GO:0060997, GO:0061564, neuron projection guidance [GO:0097485], GO:0106030